{
  "gene": "UniProtKB:Q8IXB1",
  "gene_name": "DnaJ homolog subfamily C member 10",
  "term_id": "GO:0036498",
  "term_label": "IRE1-mediated unfolded protein response",
  "gene_symbol": "DNAJC10"
}